{
  "gene_symbol": "OR2T27",
  "term_label": "plasma membrane",
  "gene_name": "Olfactory receptor 2T27",
  "term_id": "GO:0005886",
  "gene": "UniProtKB:Q8NH04"
}